{
  "term_id": "GO:0045277",
  "gene_name": "Cytochrome c oxidase subunit 4 isoform 1, mitochondrial",
  "gene": "UniProtKB:P13073",
  "gene_symbol": "COX4I1",
  "term_label": "respiratory chain complex IV"
}